{
  "term_label": "structural constituent of skin epidermis",
  "gene_symbol": "KRT33A",
  "term_id": "GO:0030280",
  "gene_name": "Keratin, type I cuticular Ha3-I",
  "gene": "UniProtKB:O76009"
}